Kv4.2-KChIP3 channel complex [GO:0071194] (cellular component) Definition: A voltage-gated potassium channel complex that contains the Kv channel interacting protein KChIP3 associated with the channel via interaction with the Kv alpha subunit 4.2. Relationships: is a type of voltage-gated potassium channel complex [GO:0008076] References: PMID:15356203